{
  "gene_symbol": "HSD17B1",
  "term_id": "GO:0004303",
  "gene": "UniProtKB:P14061",
  "gene_name": "17-beta-hydroxysteroid dehydrogenase type 1",
  "term_label": "estradiol 17-beta-dehydrogenase [NAD(P)+] activity"
}